{
  "term_label": "growth factor activity",
  "term_id": "GO:0008083",
  "gene_symbol": "FGF7",
  "gene": "UniProtKB:P21781",
  "gene_name": "Fibroblast growth factor 7"
}